{
  "term_label": "nuclear cap binding complex",
  "term_id": "GO:0005846",
  "gene": "UniProtKB:Q09161",
  "gene_name": "Nuclear cap-binding protein subunit 1",
  "gene_symbol": "NCBP1"
}